{
  "term_id": "UNKNOWN:0001",
  "gene_symbol": "MS4A3",
  "term_label": "Unknown molecular function",
  "gene_name": "Membrane-spanning 4-domains subfamily A member 3",
  "gene": "UniProtKB:Q96HJ5"
}